Golgi to plasma membrane transport vesicle [GO:0070319] (cellular component) Also known as: Golgi to plasma membrane constitutive secretory pathway transport vesicle, Golgi-plasma membrane transport vesicle Relationships: is_a exocytic vesicle [GO:0070382] Sources: GOC:kad, GOC:mah Definition: A transport vesicle that mediates transport from the Golgi to the plasma membrane, and fuses with the plasma membrane to release various cargo molecules, such as proteins or hormones, by exocytosis.